isoprenoid biosynthetic process [GO:0008299] (BP) Subtypes: prenol biosynthetic process [GO:0016091], polyprenol biosynthetic process [GO:0016094], terpenoid biosynthetic process [GO:0016114], apocarotenoid biosynthetic process [GO:0043289], terpene biosynthetic process [GO:0046246], isoprenoid biosynthetic process via mevalonate [GO:1902767], isoprenoid biosynthetic process via 1-deoxy-D-xylulose 5-phosphate [GO:1902768] Definition: The chemical reactions and pathways resulting in the formation of an isoprenoid compound, isoprene (2-methylbuta-1,3-diene) or compounds containing or derived from linked isoprene (3-methyl-2-butenylene) residues. Sources: ISBN:0198506732 Relationships: is a type of isoprenoid metabolic process [GO:0006720]; is a type of lipid biosynthetic process [GO:0008610] Also known as: isoprenoid anabolism, isoprenoid biosynthesis, isoprenoid formation, isoprenoid synthesis, polyisoprenoid anabolism, polyisoprenoid biosynthesis, polyisoprenoid biosynthetic process, polyisoprenoid formation, polyisoprenoid synthesis, polyterpene biosynthesis, polyterpene biosynthetic process